{
  "gene": "UniProtKB:O43613",
  "term_id": "GO:0004930",
  "gene_symbol": "HCRTR1",
  "term_label": "G protein-coupled receptor activity",
  "gene_name": "Orexin_Hypocretin receptor type 1"
}